{
  "gene_name": "C-C motif chemokine 21",
  "term_id": "GO:0006954",
  "gene": "UniProtKB:O00585",
  "gene_symbol": "CCL21",
  "term_label": "inflammatory response"
}